adult chitin-containing cuticle pigmentation [GO:0048085] (biological process) Relationships: is a type of GO:0048067; is part of chitin-based cuticle sclerotization [GO:0007593] Sources: GOC:jid, GOC:mtg_sensu Definition: Establishment of the adult pattern of pigmentation in the chitin-containing cuticle of an organism. An example of this is the adult cuticle pigmentation process in Drosophila melanogaster. Also known as: adult cuticle pigmentation Regulation: regulated by regulation of adult chitin-containing cuticle pigmentation [GO:0048082]; negatively regulated by negative regulation of adult chitin-containing cuticle pigmentation [GO:0048083]; positively regulated by positive regulation of adult chitin-containing cuticle pigmentation [GO:0048084]